{
  "term_id": "GO:0003743",
  "gene_symbol": "EIF4E3",
  "gene": "UniProtKB:Q8N5X7",
  "term_label": "translation initiation factor activity",
  "gene_name": "Eukaryotic translation initiation factor 4E type 3"
}